isocitrate dehydrogenase complex (NAD+) [GO:0045242] (cellular component) Sources: GOC:mah Relationships: is a type of tricarboxylic acid cycle heteromeric enzyme complex [GO:0045239]; is a type of GO:1990204 Definition: Complex that possesses isocitrate dehydrogenase (NAD+) activity.